15-hydroxyicosatetraenoate dehydrogenase activity [GO:0047034] (molecular function) Definition: Catalysis of the reaction: NAD(P)+ + (15S)-15-hydroxy-5,8,11-cis-13-trans-icosatetraenoate = NAD(P)H + H+ + 15-oxo-5,8,11-cis-13-trans-icosatetraenoate. Also known as: (15S)-15-hydroxy-5,8,11-cis-13-trans-icosatetraenoate:NAD(P)+ 15-oxidoreductase activity, 15-hydroxyeicosatetraenoate dehydrogenase activity Relationships: is a type of oxidoreductase activity, acting on the CH-OH group of donors, NAD or NADP as acceptor [GO:0016616] Sources: EC:1.1.1.232, MetaCyc:1.1.1.232-RXN